{
  "gene_symbol": "IGHV3-38-3",
  "gene": "UniProtKB:P0DTE1",
  "term_label": "antigen binding",
  "gene_name": "Probable non-functional immunoglobulin heavy variable 3-38-3",
  "term_id": "GO:0003823"
}